{
  "gene_symbol": "USP10",
  "term_label": "cytosol",
  "term_id": "GO:0005829",
  "gene_name": "Ubiquitin carboxyl-terminal hydrolase 10",
  "gene": "UniProtKB:Q14694"
}